{
  "gene": "UniProtKB:Q8WWF5",
  "term_label": "negative regulation of cell cycle",
  "gene_symbol": "ZNRF4",
  "term_id": "GO:0045786",
  "gene_name": "E3 ubiquitin-protein ligase ZNRF4"
}